{
  "term_id": "GO:0006749",
  "gene": "UniProtKB:P07203",
  "gene_symbol": "GPX1",
  "gene_name": "Glutathione peroxidase 1",
  "term_label": "glutathione metabolic process"
}